{
  "term_label": "P-body",
  "gene_symbol": "SAMD4B",
  "term_id": "GO:0000932",
  "gene": "UniProtKB:Q5PRF9",
  "gene_name": "Protein Smaug homolog 2"
}